peptide antigen assembly with MHC protein complex [GO:0002501] (biological process) Relationships: is_a protein-containing complex assembly [GO:0065003]; is part of GO:0002396; is part of GO:0048002 References: PMID:15771591 Sources: GOC:add, ISBN:0781735149 Subtypes: peptide antigen assembly with MHC class Ib protein complex [GO:0002492], peptide antigen assembly with MHC class I protein complex [GO:0002502], GO:0002503 Definition: The binding of a peptide to the antigen binding groove of an MHC protein complex.